positive regulation of tRNA catabolic process [GO:1902372] (biological process) Definition: Any process that activates or increases the frequency, rate or extent of tRNA catabolic process. Relationships: is_a GO:0009896; is a type of GO:1902370; is a type of positive regulation of tRNA metabolic process [GO:1903328]; positively regulates tRNA decay [GO:0016078] Also known as: positive regulation of tRNA breakdown, positive regulation of tRNA catabolism, positive regulation of tRNA degradation, up regulation of tRNA breakdown, up regulation of tRNA catabolic process, up regulation of tRNA catabolism, up regulation of tRNA degradation, up-regulation of tRNA breakdown, up-regulation of tRNA catabolic process, up-regulation of tRNA catabolism, up-regulation of tRNA degradation, upregulation of tRNA breakdown, upregulation of tRNA catabolic process, upregulation of tRNA catabolism, upregulation of tRNA degradation, activation of tRNA breakdown, activation of tRNA catabolic process, activation of tRNA catabolism, activation of tRNA degradation Subtypes: GO:0036417 Sources: GOC:TermGenie, GOC:bf